DNA double-strand break processing [GO:0000729] (biological process) Definition: The 5' to 3' exonucleolytic resection of the DNA at the site of the break to form a 3' single-strand DNA overhang. References: PMID:10357855 Relationships: is a type of DNA metabolic process [GO:0006259]; is part of GO:0006302; has part 5'-3' DNA exonuclease activity [GO:0035312] Subtypes: meiotic DNA double-strand break processing [GO:0000706], DNA double-strand break processing involved in repair via synthesis-dependent strand annealing [GO:0010791], DNA double-strand break processing involved in repair via single-strand annealing [GO:0010792] Regulation: regulated by regulation of DNA double-strand break processing [GO:1903775]